{
  "gene": "UniProtKB:Q14393",
  "gene_symbol": "GAS6",
  "gene_name": "Growth arrest-specific protein 6",
  "term_id": "GO:0007166",
  "term_label": "cell surface receptor signaling pathway"
}